hair cycle phase [GO:0044851] (BP) Relationships: is a type of biological phase [GO:0044848] Sources: GOC:jl Subtypes: catagen [GO:0042637], exogen [GO:0042638], telogen [GO:0042639], anagen [GO:0042640] Note: Note that this term should not be used for direct annotation. If you are trying to make an annotation to x phase, it is likely that the correct annotation is 'regulation of x/y phase transition' or to a process which occurs during the reported phase. To capture the phase when a specific location or process is observed, the phase term can be used in an annotation extension (PMID:24885854) applied to a cellular component term (with the relation exists_during) or a biological process term (with the relation happens_during). Definition: The cyclical periods of growth (anagen), regression (catagen), quiescence (telogen), and shedding (exogen) in the life of a hair; one of the collection or mass of filaments growing from the skin of an animal, and forming a covering for a part of the head or for any part or the whole of the body.